{
  "gene": "UniProtKB:Q9NRW3",
  "gene_symbol": "APOBEC3C",
  "term_label": "RNA binding",
  "term_id": "GO:0003723",
  "gene_name": "DNA dC-dU-editing enzyme APOBEC-3C"
}